{
  "gene_name": "Zinc finger protein 69 homolog",
  "gene_symbol": "ZFP69",
  "term_label": "RNA polymerase II transcription regulatory region sequence-specific DNA binding",
  "term_id": "GO:0000977",
  "gene": "UniProtKB:Q49AA0"
}